{
  "gene_symbol": "GULP1",
  "term_id": "UNKNOWN:0001",
  "gene": "UniProtKB:Q9UBP9",
  "term_label": "Unknown molecular function",
  "gene_name": "PTB domain-containing engulfment adapter protein 1"
}